positive regulation of central tolerance induction [GO:0002648] (biological process) Definition: Any process that activates or increases the frequency, rate, or extent of central tolerance induction. Sources: GOC:add Also known as: up regulation of central tolerance induction, up-regulation of central tolerance induction, upregulation of central tolerance induction, activation of central tolerance induction, stimulation of central tolerance induction Relationships: is a type of positive regulation of tolerance induction [GO:0002645]; is a type of regulation of central tolerance induction [GO:0002646]; positively regulates central tolerance induction [GO:0002508] Subtypes: positive regulation of central B cell tolerance induction [GO:0002897]